positive regulation of forward locomotion [GO:1905850] (BP) Also known as: up regulation of forward locomotion, up-regulation of forward locomotion, upregulation of forward locomotion, activation of forward locomotion References: PMID:11717360 Sources: GOC:TermGenie, GO_REF:0000058 Definition: Any process that activates or increases the frequency, rate or extent of forward locomotion. Relationships: is a type of positive regulation of locomotion [GO:0040017]; is a type of regulation of forward locomotion [GO:0043059]; positively regulates GO:0043056